{
  "gene_symbol": "DORIP1",
  "gene_name": "Uncharacterized protein C14orf28",
  "gene": "UniProtKB:Q4W4Y0",
  "term_label": "Unknown molecular function",
  "term_id": "UNKNOWN:0001"
}